{
  "gene_symbol": "SLC35D2",
  "gene_name": "UDP-N-acetylglucosamine_UDP-glucose_GDP-mannose transporter",
  "gene": "UniProtKB:Q76EJ3",
  "term_id": "GO:0015780",
  "term_label": "nucleotide-sugar transmembrane transport"
}